CUT catabolic process [GO:0071034] (BP) Also known as: cryptic unstable transcript catabolic process Subtypes: nuclear polyadenylation-dependent CUT catabolic process [GO:0071039] Sources: GOC:dgf, GOC:krc Relationships: is a type of RNA catabolic process [GO:0006401] Definition: The chemical reactions and pathways resulting in the breakdown of cryptic unstable transcripts (CUTs).